{
  "gene_name": "Acyl-coenzyme A thioesterase 6",
  "gene": "UniProtKB:Q3I5F7",
  "term_id": "GO:0047617",
  "term_label": "fatty acyl-CoA hydrolase activity",
  "gene_symbol": "ACOT6"
}